rhombomere morphogenesis [GO:0021593] (BP) Definition: The process in which the anatomical structure of the rhombomere is generated and organized. Rhombomeres are transverse segments of the developing rhombencephalon. Rhombomeres are lineage restricted, express different genes from one another, and adopt different developmental fates. Relationships: is a type of anatomical structure morphogenesis [GO:0009653]; is part of rhombomere development [GO:0021546] Subtypes: GO:0021651, GO:0021655, rhombomere 3 morphogenesis [GO:0021658], rhombomere 4 morphogenesis [GO:0021661], rhombomere 5 morphogenesis [GO:0021664], rhombomere 6 morphogenesis [GO:0021667], GO:0021671, rhombomere 8 morphogenesis [GO:0021674] Sources: GOC:cls, GOC:dgh, GOC:dph, GOC:jid, GO_REF:0000021